mesonephric podocyte cell fate commitment [GO:0061258] (biological process) Definition: The process in which the developmental fate of a cell becomes restricted such that it will develop into a mesonephric glomerular visceral epithelial cell. A mesonephric glomerular visceral epithelial cell is a specialized epithelial cell that contains 'feet' that interdigitate with the 'feet' of other glomerular epithelial cells in the mesonephros. Sources: GOC:mtg_kidney_jan10 Also known as: mesonephric glomerular visceral epithelial cell fate commitment Relationships: is a type of mesonephric glomerular epithelial cell development [GO:0061251]; is a type of GO:0072149; BFO_0000050 GO:0061256